{
  "term_id": "GO:0005886",
  "gene_symbol": "PCDHGB5",
  "term_label": "plasma membrane",
  "gene_name": "Protocadherin gamma-B5",
  "gene": "UniProtKB:Q9Y5G0"
}